anthranilate N-methyltransferase activity [GO:0030774] (molecular function) Relationships: is a type of S-adenosylmethionine-dependent methyltransferase activity [GO:0008757] Sources: EC:2.1.1.111, RHEA:12180 Definition: Catalysis of the reaction: S-adenosyl-L-methionine + anthranilate = N-methylanthranilate + S-adenosyl-L-homocysteine + H+. Also known as: S-adenosyl-L-methionine:anthranilate N-methyltransferase activity, anthranilic acid N-methyltransferase activity